{
  "gene": "UniProtKB:Q01844",
  "term_id": "UNKNOWN:0002",
  "gene_name": "RNA-binding protein EWS",
  "gene_symbol": "EWSR1",
  "term_label": "Unknown biological process"
}